dihydrofolate metabolic process [GO:0046452] (biological process) Sources: ISBN:0198506732 Definition: The chemical reactions and pathways involving dihydrofolate, the dihydroxylated derivative of folate. Subtypes: dihydrofolate biosynthetic process [GO:0006761] Also known as: dihydrofolate metabolism, dihydrofolate reduction Relationships: is_a folic acid-containing compound metabolic process [GO:0006760]; is a type of dicarboxylic acid metabolic process [GO:0043648]